symbiont-mediated perturbation of host natural killer cell mediated immune response [GO:0039671] (biological process) Definition: A process in which a symbiont alters or subverts the natural killer cell mediated immune response of the host organism. The host is defined as the larger of the organisms involved in a symbiotic interaction. References: PMID:15640804, PMID:18688275 Sources: GOC:bf, GOC:jl, UniProtKB-KW:KW-1131 Also known as: evasion by virus of host NK cell killing, evasion by virus of host natural killer cell response, protection by virus against host NK cell cytotoxicity, evasion by virus of host natural killer cell activity, suppression by virus of host natural killer cell function, viral immunoevasion of host NK cell, modulation of host NK-cell activity by virus Relationships: is a type of symbiont-mediated perturbation of host cellular process [GO:0044068]; is a type of symbiont-mediated perturbation of host innate immune response [GO:0052167] Subtypes: symbiont-mediated suppression of host natural killer cell activation [GO:0039672]